{
  "gene_symbol": "RAB10",
  "gene_name": "Ras-related protein Rab-10",
  "term_id": "GO:0055037",
  "term_label": "recycling endosome",
  "gene": "UniProtKB:P61026"
}